{
  "gene": "UniProtKB:Q8TAM2",
  "gene_symbol": "TTC8",
  "term_label": "non-motile cilium assembly",
  "gene_name": "Tetratricopeptide repeat protein 8",
  "term_id": "GO:1905515"
}